{
  "gene": "UniProtKB:Q9P202",
  "term_id": "GO:0002142",
  "gene_symbol": "WHRN",
  "term_label": "stereocilia ankle link complex",
  "gene_name": "Whirlin"
}